{
  "gene": "UniProtKB:Q0P670",
  "term_label": "Unknown molecular function",
  "term_id": "UNKNOWN:0001",
  "gene_name": "Uncharacterized protein SPEM2",
  "gene_symbol": "SPEM2"
}